HAUS complex [GO:0070652] (cellular component) References: PMID:19427217 Relationships: is a type of microtubule associated complex [GO:0005875] Also known as: HAUS augmin complex Definition: A protein complex that localizes to interphase centrosomes and to mitotic spindle tubules and regulates mitotic spindle assembly and centrosome integrity; in human, the complex consists of eight subunits, some of which are homologous to subunits of the Drosophila Augmin complex.